canonical NF-kappaB signal transduction [GO:0007249] (biological process) Relationships: is a type of intracellular signaling cassette [GO:0141124] References: PMID:12773372, PMID:34659217 Sources: GOC:bf Also known as: NF-kappaB cascade, I-kappaB kinase/NF-kappaB cascade, I-kappaB kinase/NF-kappaB signal transduction, I-kappaB kinase/NF-kappaB signaling, canonical NF-kappaB signaling cascade, p50-dependent NF-kappaB signaling Regulation: regulated by regulation of canonical NF-kappaB signal transduction [GO:0043122]; positively regulated by positive regulation of canonical NF-kappaB signal transduction [GO:0043123]; negatively regulated by negative regulation of canonical NF-kappaB signal transduction [GO:0043124] Definition: An intracellular signaling cassette characterized by the I-kappaB-kinase (IKK)-dependent activation of NF-kappaB, also known as the canonical NF-kappaB signaling cascade. The cascade begins with activation of a trimeric IKK complex (consisting of catalytic kinase subunits IKKalpha and/or IKKbeta, and the regulatory scaffold protein NEMO) and ends with the regulation of transcription of target genes by NF-kappaB. In a resting state, NF-kappaB dimers are bound to I-kappaB proteins, sequestering NF-kappaB in the cytoplasm. Phosphorylation of I-kappaB targets I-kappaB for ubiquitination and proteasomal degradation, thus releasing the NF-kappaB dimers, which can translocate to the nucleus to bind DNA and regulate transcription. The canonical NF-kappaB pathway is mainly stimulated by proinflammatory cytokines such as IL-1beta, tumor necrosis factor (TNF)-alpha, antigen ligands, and toll-like receptors (TLRs).